{
  "term_id": "GO:0000977",
  "gene_name": "Zinc finger protein 177",
  "gene_symbol": "ZNF177",
  "gene": "UniProtKB:Q13360",
  "term_label": "RNA polymerase II transcription regulatory region sequence-specific DNA binding"
}